{
  "term_label": "cytoplasm",
  "gene": "UniProtKB:Q9ULD6",
  "gene_symbol": "INTU",
  "term_id": "GO:0005737",
  "gene_name": "Protein inturned"
}